{
  "gene_symbol": "ZNF365",
  "term_id": "GO:0110026",
  "term_label": "regulation of DNA strand resection involved in replication fork processing",
  "gene": "UniProtKB:Q70YC5",
  "gene_name": "Protein ZNF365"
}